{
  "gene": "UniProtKB:A0A1B0GTU2",
  "gene_name": "Cortexin domain-containing 1 protein",
  "term_label": "Unknown molecular function",
  "term_id": "UNKNOWN:0001",
  "gene_symbol": "CTXND1"
}